{
  "term_label": "vascular endothelial growth factor binding",
  "gene": "UniProtKB:O14786",
  "gene_symbol": "NRP1",
  "term_id": "GO:0038085",
  "gene_name": "Neuropilin-1"
}